{
  "term_label": "BMP signaling pathway",
  "gene_symbol": "GDF1",
  "gene_name": "Embryonic growth_differentiation factor 1",
  "term_id": "GO:0030509",
  "gene": "UniProtKB:P27539"
}